{
  "term_id": "UNKNOWN:0002",
  "gene_symbol": "KRTAP17-1",
  "term_label": "Unknown biological process",
  "gene_name": "Keratin-associated protein 17-1",
  "gene": "UniProtKB:Q9BYP8"
}